{
  "gene": "UniProtKB:Q8N957",
  "term_id": "UNKNOWN:0001",
  "gene_symbol": "ANKFN1",
  "gene_name": "Ankyrin repeat and fibronectin type-III domain-containing protein 1",
  "term_label": "Unknown molecular function"
}